mitochondrial translation preinitiation complex [GO:0180053] (cellular component) Definition: A ribonucleoprotein complex comprising of the 28S small mitoribosomal subunit (mt-SSU) and mitochondrial initiation factors (e.g. mtIF3 and mtIF2-GTP) and the initiator tRNA-Met and an mRNA binding. The early steps of translation initiation, including the association of the 28S mitochondrial small subunit (mt-SSU) with initiation factors (mtIF3 and mtIF2), prevention of premature large subunit (39S) joining occur during the assembly of the mitochondrial pre-initiation complex (mtPIC). Also known as: mitochondrial translation pre-initiation complex Relationships: is a type of mitochondrial protein-containing complex [GO:0098798]; is a type of ribonucleoprotein complex [GO:1990904]; is part of mitochondrial matrix [GO:0005759] References: PMID:32522994 Sources: GOC:vw